{
  "gene": "UniProtKB:Q9UPQ3",
  "term_label": "GTPase activity",
  "gene_name": "Arf-GAP with GTPase, ANK repeat and PH domain-containing protein 1",
  "term_id": "GO:0003924",
  "gene_symbol": "AGAP1"
}